{
  "gene_name": "Villin-like protein",
  "term_id": "GO:0051015",
  "gene_symbol": "VILL",
  "gene": "UniProtKB:O15195",
  "term_label": "actin filament binding"
}